{
  "gene_name": "ABC-type oligopeptide transporter ABCB9",
  "gene": "UniProtKB:Q9NP78",
  "term_id": "GO:0015440",
  "gene_symbol": "ABCB9",
  "term_label": "ABC-type peptide transporter activity"
}